{
  "gene": "UniProtKB:A0A0A0MT89",
  "term_id": "UNKNOWN:0003",
  "term_label": "Unknown cellular component",
  "gene_symbol": "IGKJ1",
  "gene_name": "Immunoglobulin kappa joining 1"
}